{
  "gene_name": "SLIT and NTRK-like protein 5",
  "term_id": "UNKNOWN:0003",
  "term_label": "Unknown cellular component",
  "gene_symbol": "SLITRK5",
  "gene": "UniProtKB:O94991"
}